galactosylceramide sulfotransferase activity [GO:0001733] (molecular function) Definition: Catalysis of the reaction: 3'-phosphoadenosine 5'-phosphosulfate + a galactosylceramide = adenosine 3',5'-bisphosphate + a galactosylceramidesulfate. Relationships: is a type of galactose 3-O-sulfotransferase activity [GO:0050694] Also known as: cerebroside sulfotransferase activity, galactosylceramide sulphotransferase activity, 3'-phosphoadenosine-5'-phosphosulfate-cerebroside sulfotransferase activity, 3'-phosphoadenylyl-sulfate:galactosylceramide 3'-sulfotransferase activity, GSase, galactocerebroside sulfotransferase activity, galactolipid sulfotransferase activity, glycolipid sulfotransferase activity, glycosphingolipid sulfotransferase activity References: PMID:10727929 Sources: EC:2.8.2.11, RHEA:20613